{
  "gene_name": "Trafficking protein particle complex subunit 4",
  "term_label": "Unknown molecular function",
  "gene": "UniProtKB:Q9Y296",
  "gene_symbol": "TRAPPC4",
  "term_id": "UNKNOWN:0001"
}